{
  "term_id": "GO:0034976",
  "gene_name": "E3 ubiquitin-protein ligase RNF183",
  "gene_symbol": "RNF183",
  "term_label": "response to endoplasmic reticulum stress",
  "gene": "UniProtKB:Q96D59"
}